regulation of myeloid dendritic cell antigen processing and presentation [GO:0002607] (biological process) Relationships: is a type of regulation of dendritic cell antigen processing and presentation [GO:0002604]; regulates myeloid dendritic cell antigen processing and presentation [GO:0002469] Sources: GOC:add Definition: Any process that modulates the frequency, rate, or extent of myeloid dendritic cell antigen processing and presentation. Subtypes: GO:0002608, positive regulation of myeloid dendritic cell antigen processing and presentation [GO:0002609]